{
  "gene": "UniProtKB:P22914",
  "gene_symbol": "CRYGS",
  "term_id": "GO:0005212",
  "term_label": "structural constituent of eye lens",
  "gene_name": "Gamma-crystallin S"
}